protein O-linked glycosylation via fucose [GO:0036066] (BP) References: PMID:16899492, PMID:35536928 Definition: A glycoprotein biosynthetic process starting with the covalent linkage of a fucose via an alpha-glycosidic bond to the oxygen atom of a serine or threonine side chain in a protein, which can be further elongated with the sequential addition of sugar units resulting in the formation of a protein O-linked glycan. This modification typically occurs within specific motifs, such as EGF-like or thrombospondin type-1 repeats. Also known as: protein O-linked fucosylation Relationships: is_a protein O-linked glycosylation [GO:0006493]